{
  "gene": "UniProtKB:P00736",
  "term_label": "extracellular space",
  "term_id": "GO:0005615",
  "gene_symbol": "C1R",
  "gene_name": "Complement C1r subcomponent"
}